{
  "gene_name": "Insulinoma-associated protein 2",
  "gene_symbol": "INSM2",
  "term_id": "GO:0010564",
  "term_label": "regulation of cell cycle process",
  "gene": "UniProtKB:Q96T92"
}